positive regulation of spontaneous neurotransmitter secretion [GO:1904050] (BP) Note: An example of this is PARK2 / parkin in human (O60260) in PMID:22314364 (inferred from mutant phenotype). Also known as: positive regulation of stimulus-independent neurotransmitter secretion, up regulation of spontaneous neurotransmitter secretion, up regulation of stimulus-independent neurotransmitter secretion, up-regulation of spontaneous neurotransmitter secretion, up-regulation of stimulus-independent neurotransmitter secretion, upregulation of spontaneous neurotransmitter secretion, upregulation of stimulus-independent neurotransmitter secretion, activation of spontaneous neurotransmitter secretion, activation of stimulus-independent neurotransmitter secretion Relationships: is_a positive regulation of neurotransmitter secretion [GO:0001956]; is a type of regulation of spontaneous neurotransmitter secretion [GO:1904048]; positively regulates spontaneous neurotransmitter secretion [GO:0061669] References: PMID:22314364 Sources: GOC:PARL, GOC:TermGenie, GOC:pad, GO_REF:0000058 Definition: Any process that activates or increases the frequency, rate or extent of spontaneous neurotransmitter secretion.